{
  "gene": "UniProtKB:O15544",
  "gene_name": "Protein GR6",
  "term_id": "UNKNOWN:0003",
  "gene_symbol": "LINC01565",
  "term_label": "Unknown cellular component"
}